{
  "gene": "UniProtKB:Q9H009",
  "gene_name": "Nascent polypeptide-associated complex subunit alpha-2",
  "term_id": "GO:0005737",
  "gene_symbol": "NACA2",
  "term_label": "cytoplasm"
}